{
  "gene": "UniProtKB:Q8N205",
  "term_label": "Unknown molecular function",
  "gene_name": "Nesprin-4",
  "term_id": "UNKNOWN:0001",
  "gene_symbol": "SYNE4"
}